leukotriene B4 metabolic process [GO:0036102] (biological process) Definition: The chemical reactions and pathways involving leukotriene B4, a leukotriene composed of (6Z,8E,10E,14Z)-eicosatetraenoic acid having (5S)- and (12R)-hydroxy substituents. Sources: GOC:bf Also known as: LTB4 metabolism Relationships: is a type of long-chain fatty acid metabolic process [GO:0001676]; is a type of leukotriene metabolic process [GO:0006691]; is a type of fatty acid derivative metabolic process [GO:1901568] Subtypes: GO:0036101, GO:0097251